{
  "gene": "UniProtKB:Q86UX2",
  "term_label": "Unknown biological process",
  "term_id": "UNKNOWN:0002",
  "gene_name": "Inter-alpha-trypsin inhibitor heavy chain H5",
  "gene_symbol": "ITIH5"
}